{
  "gene": "UniProtKB:O43663",
  "term_id": "GO:0000226",
  "gene_name": "Protein regulator of cytokinesis 1",
  "gene_symbol": "PRC1",
  "term_label": "microtubule cytoskeleton organization"
}